head kidney maturation [GO:0072121] (biological process) Sources: GOC:mtg_kidney_jan10, ZFA:0000669 Relationships: is a type of pronephros maturation [GO:0072120]; is part of head kidney development [GO:0072113] Definition: A developmental process, independent of morphogenetic (shape) change, that is required for the head kidney to attain its fully functional state. The head kidney is a pronephros that consists of fused bilateral lobes located in the anterior part of the kidney.